{
  "gene_name": "Putative small nuclear ribonucleoprotein G-like protein 15",
  "gene_symbol": "SNRPGP15",
  "term_label": "RNA binding",
  "gene": "UniProtKB:A8MWD9",
  "term_id": "GO:0003723"
}